alcohol binding [GO:0043178] (molecular function) Subtypes: inositol hexakisphosphate binding [GO:0000822], GO:0010427, cholesterol binding [GO:0015485], GO:0019841, GO:0030975, hydroxyectoine binding [GO:0033295], GO:0035100, ethanol binding [GO:0035276], GO:0043533, inositol 1,4,5 trisphosphate binding [GO:0070679], GO:1903794, corticosterone binding [GO:1903875], 11-deoxycortisol binding [GO:1903876], 21-deoxycortisol binding [GO:1903877], 11-deoxycorticosterone binding [GO:1903878], GO:1903880 Sources: GOC:jl, ISBN:0198506732 Definition: Binding to an alcohol, any of a class of alkyl compounds containing a hydroxyl group. Relationships: is a type of small molecule binding [GO:0036094]